{
  "gene": "UniProtKB:Q9Y5G1",
  "gene_name": "Protocadherin gamma-B3",
  "term_label": "cell adhesion molecule binding",
  "term_id": "GO:0050839",
  "gene_symbol": "PCDHGB3"
}